{
  "gene": "UniProtKB:Q8NHP1",
  "term_id": "GO:0008106",
  "gene_name": "Aflatoxin B1 aldehyde reductase member 4",
  "gene_symbol": "AKR7L",
  "term_label": "alcohol dehydrogenase (NADP+) activity"
}